{
  "term_label": "Unknown cellular component",
  "term_id": "UNKNOWN:0003",
  "gene": "UniProtKB:Q6P4F7",
  "gene_symbol": "ARHGAP11A",
  "gene_name": "Rho GTPase-activating protein 11A"
}